DNA-binding transcription repressor activity, RNA polymerase III-specific [GO:0106250] (molecular function) Definition: A DNA-binding transcription factor activity that represses or decreases the transcription of specific genes sets transcribed by RNA polymerase III. References: PMID:15590667, PMID:31833215 Sources: GOC:txnOH-2018 Note: For usage guidance, see comment in GO:0003700 ; DNA-binding transcription factor activity. Relationships: is a type of DNA-binding transcription repressor activity [GO:0001217]; is part of negative regulation of transcription by RNA polymerase III [GO:0016480]; has part RNA polymerase III transcription regulatory region sequence-specific DNA binding [GO:0001016]; occurs in chromatin [GO:0000785]